{
  "gene_name": "Homocysteine-responsive endoplasmic reticulum-resident ubiquitin-like domain member 1 protein",
  "term_id": "GO:0032469",
  "gene": "UniProtKB:Q15011",
  "term_label": "endoplasmic reticulum calcium ion homeostasis",
  "gene_symbol": "HERPUD1"
}